{
  "gene_name": "Thromboxane-A synthase",
  "gene_symbol": "TBXAS1",
  "gene": "UniProtKB:P24557",
  "term_id": "UNKNOWN:0003",
  "term_label": "Unknown cellular component"
}